{
  "gene_name": "Zinc finger protein DPF3",
  "gene_symbol": "DPF3",
  "gene": "UniProtKB:Q92784",
  "term_id": "GO:0005634",
  "term_label": "nucleus"
}